{
  "gene_symbol": "ETV6",
  "gene_name": "Transcription factor ETV6",
  "gene": "UniProtKB:P41212",
  "term_id": "GO:0005634",
  "term_label": "nucleus"
}